nitric oxide transmembrane transporter activity [GO:0030184] (MF) Definition: Enables the transfer of nitric oxide, nitrogen monoxide, from one side of a membrane to the other. Sources: GOC:mah Relationships: is a type of transmembrane transporter activity [GO:0022857]; is part of nitric oxide transport [GO:0030185]